{
  "term_id": "GO:0045665",
  "gene_symbol": "HES1",
  "gene_name": "Transcription factor HES-1",
  "term_label": "negative regulation of neuron differentiation",
  "gene": "UniProtKB:Q14469"
}